{
  "term_id": "UNKNOWN:0001",
  "term_label": "Unknown molecular function",
  "gene": "UniProtKB:Q9NV12",
  "gene_name": "Transmembrane protein 140",
  "gene_symbol": "TMEM140"
}